{
  "gene_name": "Kinesin-like protein KIF3B",
  "term_label": "microtubule motor activity",
  "term_id": "GO:0003777",
  "gene_symbol": "KIF3B",
  "gene": "UniProtKB:O15066"
}